{
  "term_label": "Unknown cellular component",
  "gene_symbol": "GALNT1",
  "gene": "UniProtKB:Q10472",
  "gene_name": "Polypeptide N-acetylgalactosaminyltransferase 1",
  "term_id": "UNKNOWN:0003"
}